{
  "term_label": "Unknown biological process",
  "gene": "UniProtKB:Q9P109",
  "term_id": "UNKNOWN:0002",
  "gene_symbol": "GCNT4",
  "gene_name": "Beta-1,3-galactosyl-O-glycosyl-glycoprotein beta-1,6-N-acetylglucosaminyltransferase 4"
}